{
  "gene_name": "Glutamyl-tRNA(Gln) amidotransferase subunit A, mitochondrial",
  "gene_symbol": "QRSL1",
  "term_label": "glutaminyl-tRNA synthase (glutamine-hydrolyzing) activity",
  "term_id": "GO:0050567",
  "gene": "UniProtKB:Q9H0R6"
}